{
  "gene_symbol": "GPC4",
  "gene_name": "Glypican-4",
  "term_label": "regulation of presynapse assembly",
  "gene": "UniProtKB:O75487",
  "term_id": "GO:1905606"
}